{
  "term_label": "Unknown molecular function",
  "gene_symbol": "SYNGR2",
  "gene": "UniProtKB:O43760",
  "gene_name": "Synaptogyrin-2",
  "term_id": "UNKNOWN:0001"
}